{
  "term_label": "nucleotide-excision repair",
  "gene_name": "Replication protein A 14 kDa subunit",
  "term_id": "GO:0006289",
  "gene_symbol": "RPA3",
  "gene": "UniProtKB:P35244"
}